{
  "gene": "UniProtKB:Q659A1",
  "gene_symbol": "ICE2",
  "term_id": "UNKNOWN:0003",
  "term_label": "Unknown cellular component",
  "gene_name": "Little elongation complex subunit 2"
}